{
  "gene_name": "Olfactory receptor 10H5",
  "term_id": "GO:0004984",
  "term_label": "olfactory receptor activity",
  "gene_symbol": "OR10H5",
  "gene": "UniProtKB:Q8NGA6"
}